purine nucleotide transmembrane transporter activity [GO:0015216] (MF) Subtypes: adenine nucleotide transmembrane transporter activity [GO:0000295], guanine nucleotide transmembrane transporter activity [GO:0001409], purine ribonucleotide transmembrane transporter activity [GO:0005346], GO:0160042 Sources: GOC:ai Relationships: is a type of nucleotide transmembrane transporter activity [GO:0015215]; is part of purine nucleotide transport [GO:0015865] Definition: Enables the transfer of a purine nucleotide, any compound consisting of a purine nucleoside esterified with (ortho)phosphate, from one side of a membrane to the other.